{
  "gene_name": "Transmembrane protein 204",
  "gene": "UniProtKB:Q9BSN7",
  "term_label": "smooth muscle cell differentiation",
  "gene_symbol": "TMEM204",
  "term_id": "GO:0051145"
}